{
  "term_id": "GO:0000775",
  "gene_name": "Sister chromatid cohesion protein DCC1",
  "gene_symbol": "DSCC1",
  "gene": "UniProtKB:Q9BVC3",
  "term_label": "chromosome, centromeric region"
}